{
  "gene_symbol": "DCD",
  "term_id": "GO:0005615",
  "term_label": "extracellular space",
  "gene": "UniProtKB:P81605",
  "gene_name": "Dermcidin"
}